positive regulation of filamentous growth of a population of unicellular organisms in response to neutral pH [GO:1900442] (biological process) Relationships: is a type of GO:1900440; is a type of positive regulation of filamentous growth of a population of unicellular organisms in response to pH [GO:1900743]; positively regulates filamentous growth of a population of unicellular organisms in response to neutral pH [GO:0036178] Sources: GOC:TermGenie, GOC:di Also known as: up regulation of filamentous growth of a population of unicellular organisms in response to neutral pH, up-regulation of filamentous growth of a population of unicellular organisms in response to neutral pH, upregulation of filamentous growth of a population of unicellular organisms in response to neutral pH, activation of filamentous growth of a population of unicellular organisms in response to neutral pH Definition: Any process that activates or increases the frequency, rate or extent of filamentous growth of a population of unicellular organisms in response to neutral pH.